cellular response to granulocyte macrophage colony-stimulating factor stimulus [GO:0097011] (biological process) Definition: Any process that results in a change in state or activity of a cell (in terms of movement, secretion, enzyme production, gene expression, etc.) as a result of a granulocyte macrophage colony-stimulating factor stimulus. References: PMID:7901744 Sources: GOC:BHF, GOC:ebc Also known as: cellular response to GM-CSF stimulus Relationships: is a type of cellular response to cytokine stimulus [GO:0071345]; is a type of GO:0097012